{
  "term_label": "extracellular space",
  "term_id": "GO:0005615",
  "gene": "UniProtKB:P51884",
  "gene_symbol": "LUM",
  "gene_name": "Lumican"
}